glutamate decarboxylase complex [GO:1902793] (cellular component) Definition: A protein complex which is capable of glutamate decarboxylase activity. References: PMID:17384644 Sources: GOC:TermGenie, GOC:bhm, GO_REF:0000088 Note: An example of this is GAD1 in human (Q99259) in PMID:17384644 (inferred from direct assay). Relationships: is a type of catalytic complex [GO:1902494]